butyrate metabolic process [GO:0019605] (biological process) Also known as: butanoic acid metabolic process, butanoic acid metabolism, butyrate metabolism, butyric acid metabolic process, butyric acid metabolism Definition: The chemical reactions and pathways involving any butyrate, the anions of butyric acid (butanoic acid), a saturated, unbranched aliphatic acid. Subtypes: glucose catabolic process to butyrate [GO:0030645], GO:0033508, butyrate biosynthetic process [GO:0046358], butyrate catabolic process [GO:0046359] Relationships: is a type of short-chain fatty acid metabolic process [GO:0046459] Sources: ISBN:0198506732